histone H3K36 methyltransferase activity [GO:0046975] (molecular function) Definition: Catalysis of the reaction: S-adenosyl-L-methionine + histone H3 L-lysine (position 36) = S-adenosyl-L-homocysteine + histone H3 N6-methyl-L-lysine (position 36). This reaction is the addition of a methyl group to the lysine residue at position 36 of the histone H3 protein. Relationships: is_a protein-lysine N-methyltransferase activity [GO:0016279]; is a type of histone H3 methyltransferase activity [GO:0140938] Also known as: histone H3K36 methylase activity, histone lysine N-methyltransferase activity (H3-K36 specific), histone methylase activity (H3-K36 specific), histone methyltransferase activity (H3-K36 specific), histone-H3K36 methyltransferase activity Sources: GOC:ai Note: Comment: Note that the residue position corresponds to the canonical human H3 histone (UniProtKB:P84243); this residue is conserved across all eukaryotes. Residue 1 is the first residue following removal of the initiating Methionine (Met). Note that each histone is encoded by multiple genes, and sequences may vary across different genes within an organism. Subtypes: GO:0140954, histone H3K36 trimethyltransferase activity [GO:0140955]